beta-primeverosidase activity [GO:0050535] (MF) Definition: Catalysis of the reaction: a 6-O-(beta-D-xylopyranosyl)-beta-D-glucopyranoside + H2O = 6-O-(beta-D-xylopyranosyl)-beta-D-glucopyranose + an alcohol. Relationships: is_a GO:0004553 Also known as: b-primeverosidase activity, 6-O-(beta-D-xylopyranosyl)-beta-D-glucopyranoside 6-O-(beta-D-xylosyl)-beta-D-glucohydrolase activity Sources: RHEA:24480